{
  "gene": "UniProtKB:Q9P0S2",
  "term_label": "mitochondrial respiratory chain complex IV assembly",
  "term_id": "GO:0033617",
  "gene_name": "Cytochrome c oxidase assembly protein COX16 homolog, mitochondrial",
  "gene_symbol": "COX16"
}